positive regulation of iodide transmembrane transport [GO:1904214] (biological process) Definition: Any process that activates or increases the frequency, rate or extent of iodide transmembrane transport. Also known as: up regulation of iodide transmembrane transport, up-regulation of iodide transmembrane transport, upregulation of iodide transmembrane transport, activation of iodide transmembrane transport References: PMID:20392814 Sources: GOC:TermGenie, GO_REF:0000058 Relationships: is_a positive regulation of anion transmembrane transport [GO:1903961]; is a type of positive regulation of iodide transport [GO:1904203]; is a type of GO:1904212; positively regulates GO:1904200